{
  "term_id": "GO:0005886",
  "gene_symbol": "APBA3",
  "term_label": "plasma membrane",
  "gene": "UniProtKB:O96018",
  "gene_name": "Amyloid-beta A4 precursor protein-binding family A member 3"
}